{
  "gene_symbol": "MAP1S",
  "gene": "UniProtKB:Q66K74",
  "term_label": "microtubule",
  "term_id": "GO:0005874",
  "gene_name": "Microtubule-associated protein 1S"
}